{
  "term_label": "Unknown molecular function",
  "gene_symbol": "LRP5L",
  "term_id": "UNKNOWN:0001",
  "gene_name": "Low-density lipoprotein receptor-related protein 5-like protein",
  "gene": "UniProtKB:A4QPB2"
}